{
  "gene_symbol": "RNF19B",
  "term_id": "GO:0000151",
  "gene_name": "E3 ubiquitin-protein ligase RNF19B",
  "gene": "UniProtKB:Q6ZMZ0",
  "term_label": "ubiquitin ligase complex"
}